{
  "gene": "UniProtKB:Q8IZQ8",
  "term_label": "cardiac muscle cell differentiation",
  "gene_name": "Myocardin",
  "term_id": "GO:0055007",
  "gene_symbol": "MYOCD"
}